{
  "gene_symbol": "LOXL3",
  "term_label": "protein-lysine 6-oxidase activity",
  "gene_name": "Lysyl oxidase homolog 3",
  "gene": "UniProtKB:P58215",
  "term_id": "GO:0004720"
}